{
  "gene": "UniProtKB:Q8IX04",
  "term_label": "ESCRT I complex",
  "term_id": "GO:0000813",
  "gene_name": "Ubiquitin-conjugating enzyme E2 variant 3",
  "gene_symbol": "UEVLD"
}